{
  "gene": "UniProtKB:Q8IZU1",
  "gene_name": "Protein FAM9A",
  "term_label": "meiotic cell cycle",
  "gene_symbol": "FAM9A",
  "term_id": "GO:0051321"
}